{
  "term_label": "DNA-binding transcription factor activity, RNA polymerase II-specific",
  "term_id": "GO:0000981",
  "gene_name": "Myogenic factor 5",
  "gene_symbol": "MYF5",
  "gene": "UniProtKB:P13349"
}